{
  "gene_name": "Phospholipase A2 group V",
  "term_id": "GO:0042130",
  "term_label": "negative regulation of T cell proliferation",
  "gene": "UniProtKB:P39877",
  "gene_symbol": "PLA2G5"
}